{
  "gene_name": "Epiplakin",
  "gene": "UniProtKB:P58107",
  "gene_symbol": "EPPK1",
  "term_id": "GO:0005737",
  "term_label": "cytoplasm"
}